{
  "gene_symbol": "IDI2-AS1",
  "gene_name": "Uncharacterized protein IDI2-AS1",
  "gene": "UniProtKB:Q9NZ38",
  "term_label": "Unknown cellular component",
  "term_id": "UNKNOWN:0003"
}